{
  "term_id": "GO:0015459",
  "gene": "UniProtKB:Q14722",
  "term_label": "potassium channel regulator activity",
  "gene_name": "Voltage-gated potassium channel subunit beta-1",
  "gene_symbol": "KCNAB1"
}